positive regulation of P-type sodium:potassium-exchanging transporter activity [GO:1903408] (biological process) Relationships: is_a positive regulation of ATP-dependent activity [GO:0032781]; is a type of regulation of P-type sodium:potassium-exchanging transporter activity [GO:1903406]; is a type of positive regulation of sodium ion transmembrane transporter activity [GO:2000651]; RO_0002213 P-type sodium:potassium-exchanging transporter activity [GO:0005391] Definition: Any process that activates or increases the frequency, rate or extent of sodium:potassium-exchanging ATPase activity. References: PMID:8160880 Sources: GOC:TermGenie, GOC:mr, GO_REF:0000059 Also known as: positive regulation of (Na+ + K+)-ATPase activity, positive regulation of (Na+ + K+)-activated ATPase activity, positive regulation of ATP phosphohydrolase (Na+/K+-exchanging), positive regulation of Na(+)/K(+)-ATPase activity, positive regulation of Na(+)/K(+)-exchanging ATPase activity, positive regulation of Na+,K+-ATPase activity, positive regulation of Na+/K+-ATPase activity, positive regulation of Na+/K+-exchanging ATPase activity, positive regulation of Na,K-activated ATPase activity, positive regulation of sodium/potassium-exchanging ATPase activity, positive regulation of sodium/potassium-transporting ATPase activity, positive regulation of sodium:potassium exchanging ATPase activity, positive regulation of sodium:potassium-exchanging ATPase activity, up regulation of (Na+ + K+)-ATPase activity, up regulation of (Na+ + K+)-activated ATPase activity, up regulation of ATP phosphohydrolase (Na+/K+-exchanging), up regulation of Na(+)/K(+)-ATPase activity, up regulation of Na(+)/K(+)-exchanging ATPase activity, up regulation of Na+,K+-ATPase activity, up regulation of Na+/K+-ATPase activity, up regulation of Na+/K+-exchanging ATPase activity, up regulation of Na,K-activated ATPase activity, up regulation of sodium/potassium-exchanging ATPase activity, up regulation of sodium/potassium-transporting ATPase activity, up regulation of sodium:potassium exchanging ATPase activity, up regulation of sodium:potassium-exchanging ATPase activity, up-regulation of (Na+ + K+)-ATPase activity, up-regulation of (Na+ + K+)-activated ATPase activity, up-regulation of ATP phosphohydrolase (Na+/K+-exchanging), up-regulation of Na(+)/K(+)-ATPase activity, up-regulation of Na(+)/K(+)-exchanging ATPase activity, up-regulation of Na+,K+-ATPase activity, up-regulation of Na+/K+-ATPase activity, up-regulation of Na+/K+-exchanging ATPase activity, up-regulation of Na,K-activated ATPase activity, up-regulation of sodium/potassium-exchanging ATPase activity, up-regulation of sodium/potassium-transporting ATPase activity, up-regulation of sodium:potassium exchanging ATPase activity, up-regulation of sodium:potassium-exchanging ATPase activity, upregulation of (Na+ + K+)-ATPase activity, upregulation of (Na+ + K+)-activated ATPase activity, upregulation of ATP phosphohydrolase (Na+/K+-exchanging), upregulation of Na(+)/K(+)-ATPase activity, upregulation of Na(+)/K(+)-exchanging ATPase activity, upregulation of Na+,K+-ATPase activity, upregulation of Na+/K+-ATPase activity, upregulation of Na+/K+-exchanging ATPase activity, upregulation of Na,K-activated ATPase activity, upregulation of sodium/potassium-exchanging ATPase activity, upregulation of sodium/potassium-transporting ATPase activity, upregulation of sodium:potassium exchanging ATPase activity, upregulation of sodium:potassium-exchanging ATPase activity, activation of (Na+ + K+)-ATPase activity, activation of (Na+ + K+)-activated ATPase activity, activation of ATP phosphohydrolase (Na+/K+-exchanging), activation of Na(+)/K(+)-ATPase activity, activation of Na(+)/K(+)-exchanging ATPase activity, activation of Na+,K+-ATPase activity, activation of Na+/K+-ATPase activity, activation of Na+/K+-exchanging ATPase activity, activation of Na,K-activated ATPase activity, activation of sodium/potassium-exchanging ATPase activity, activation of sodium/potassium-transporting ATPase activity, activation of sodium:potassium exchanging ATPase activity, activation of sodium:potassium-exchanging ATPase activity, activation of Na+,K+ pump, activation of Na,K-pump, positive regulation of Na+,K+ pump, positive regulation of Na,K-pump, up regulation of Na+,K+ pump, up regulation of Na,K-pump, up-regulation of Na+,K+ pump, up-regulation of Na,K-pump, upregulation of Na+,K+ pump, upregulation of Na,K-pump